{
  "term_label": "Unknown biological process",
  "term_id": "UNKNOWN:0002",
  "gene": "UniProtKB:Q5T5N4",
  "gene_symbol": "C6orf118",
  "gene_name": "Uncharacterized protein C6orf118"
}